{
  "term_id": "GO:0005886",
  "gene_symbol": "GRM1",
  "term_label": "plasma membrane",
  "gene_name": "Metabotropic glutamate receptor 1",
  "gene": "UniProtKB:Q13255"
}